extracellular region [GO:0005576] (cellular component) Sources: GOC:go_curators Also known as: extracellular Relationships: is a type of GO:0110165 Subtypes: GO:0043083, apoplast [GO:0048046], perivitelline space [GO:0098595], GO:0099544 Note: Note that this term is intended to annotate gene products that are not attached to the cell surface. For gene products from multicellular organisms which are secreted from a cell but retained within the organism (i.e. released into the interstitial fluid or blood), consider the cellular component term 'extracellular space ; GO:0005615'. Definition: The space external to the outermost structure of a cell. For cells without external protective or external encapsulating structures this refers to space outside of the plasma membrane. This term covers the host cell environment outside an intracellular parasite.